coenzyme A biosynthetic process [GO:0015937] (biological process) Definition: The chemical reactions and pathways resulting in the formation of coenzyme A, 3'-phosphoadenosine-(5')diphospho(4')pantatheine, an acyl carrier in many acylation and acyl-transfer reactions in which the intermediate is a thiol ester. Relationships: is a type of coenzyme A metabolic process [GO:0015936]; is a type of amide biosynthetic process [GO:0043604]; is a type of sulfur compound biosynthetic process [GO:0044272]; is a type of purine-containing compound biosynthetic process [GO:0072522]; is a type of GO:1901293 Regulation: regulated by GO:0080020 Sources: ISBN:0198547684 Also known as: CoA biosynthesis, coenzyme A anabolism, coenzyme A biosynthesis, coenzyme A formation, coenzyme A synthesis